mitotic cleavage furrow formation [GO:1903673] (biological process) Definition: Any cleavage furrow formation that is involved in mitotic cell cycle. Also known as: cleavage furrow positioning involved in mitotic cell cycle Sources: GOC:TermGenie, GOC:mtg_cell_cycle, GO_REF:0000060 Relationships: is a type of cleavage furrow formation [GO:0036089]; is a type of mitotic cytokinetic process [GO:1902410]